{
  "gene_name": "FLYWCH-type zinc finger-containing protein 1",
  "gene": "UniProtKB:Q4VC44",
  "gene_symbol": "FLYWCH1",
  "term_label": "Unknown cellular component",
  "term_id": "UNKNOWN:0003"
}